positive regulation of B cell cytokine production [GO:0002723] (biological process) Also known as: positive regulation of B lymphocyte cytokine production, positive regulation of B-cell cytokine production, positive regulation of B-lymphocyte cytokine production, up regulation of B cell cytokine production, up-regulation of B cell cytokine production, upregulation of B cell cytokine production, activation of B cell cytokine production, stimulation of B cell cytokine production Sources: GOC:add Definition: Any process that activates or increases the frequency, rate, or extent of B cell cytokine production. Relationships: is a type of positive regulation of B cell mediated immunity [GO:0002714]; is_a positive regulation of cytokine production involved in immune response [GO:0002720]; is a type of regulation of B cell cytokine production [GO:0002721]; positively regulates B cell cytokine production [GO:0002368]